{
  "term_label": "meiotic DNA integrity checkpoint signaling",
  "term_id": "GO:0044778",
  "gene_symbol": "HUS1B",
  "gene": "UniProtKB:Q8NHY5",
  "gene_name": "Checkpoint protein HUS1B"
}